{
  "term_id": "GO:0003924",
  "gene_symbol": "GBP2",
  "term_label": "GTPase activity",
  "gene": "UniProtKB:P32456",
  "gene_name": "Guanylate-binding protein 2"
}